{
  "gene_name": "Follicle-stimulating hormone receptor",
  "term_label": "plasma membrane",
  "term_id": "GO:0005886",
  "gene": "UniProtKB:P23945",
  "gene_symbol": "FSHR"
}